{
  "term_id": "UNKNOWN:0002",
  "term_label": "Unknown biological process",
  "gene_symbol": "CCDC195",
  "gene": "UniProtKB:A0A1B0GUA6",
  "gene_name": "Putative coiled-coil domain-containing protein 195"
}